benzodiazepine receptor activity [GO:0008503] (molecular function) Note: Note that this term represents an activity and not a gene product. Consider also annotating to the molecular function terms 'chloride channel activity ; GO:0005254', 'GABA receptor activity ; GO:0016917' and 'inhibitory extracellular ligand-gated ion channel activity ; GO:0005237'. Sources: GOC:jl Definition: Combining with benzodiazepines, a class of drugs with hypnotic, anxiolytic, anticonvulsive, amnestic and myorelaxant properties, to initiate a change in cell activity. Relationships: is a type of neurotransmitter receptor activity [GO:0030594]